platelet-derived growth factor binding [GO:0048407] (molecular function) Sources: GOC:dgh Definition: Binding to platelet-derived growth factor. Relationships: is a type of growth factor binding [GO:0019838] Also known as: PDGF binding